negative regulation of tetrapyrrole biosynthetic process [GO:1901464] (biological process) Relationships: is a type of negative regulation of biosynthetic process [GO:0009890]; is a type of regulation of tetrapyrrole biosynthetic process [GO:1901463]; negatively regulates tetrapyrrole biosynthetic process [GO:0033014] Definition: Any process that stops, prevents or reduces the frequency, rate or extent of tetrapyrrole biosynthetic process. Also known as: down regulation of tetrapyrrole anabolism, down regulation of tetrapyrrole biosynthesis, down regulation of tetrapyrrole biosynthetic process, down regulation of tetrapyrrole formation, down regulation of tetrapyrrole synthesis, down-regulation of tetrapyrrole anabolism, down-regulation of tetrapyrrole biosynthesis, down-regulation of tetrapyrrole biosynthetic process, down-regulation of tetrapyrrole formation, down-regulation of tetrapyrrole synthesis, downregulation of tetrapyrrole anabolism, downregulation of tetrapyrrole biosynthesis, downregulation of tetrapyrrole biosynthetic process, downregulation of tetrapyrrole formation, downregulation of tetrapyrrole synthesis, inhibition of tetrapyrrole anabolism, inhibition of tetrapyrrole biosynthesis, inhibition of tetrapyrrole formation, inhibition of tetrapyrrole synthesis, negative regulation of tetrapyrrole anabolism, negative regulation of tetrapyrrole biosynthesis, negative regulation of tetrapyrrole formation, negative regulation of tetrapyrrole synthesis, inhibition of tetrapyrrole biosynthetic process Sources: GOC:TermGenie, GOC:mengo_curators Subtypes: negative regulation of heme biosynthetic process [GO:0070454], negative regulation of tetrapyrrole biosynthetic process from glutamate [GO:1901411], GO:1901414, GO:1902325